{
  "gene": "UniProtKB:O14949",
  "term_label": "Unknown molecular function",
  "gene_name": "Cytochrome b-c1 complex subunit 8",
  "term_id": "UNKNOWN:0001",
  "gene_symbol": "UQCRQ"
}